{
  "term_id": "UNKNOWN:0003",
  "term_label": "Unknown cellular component",
  "gene_name": "Hippocampus abundant transcript 1 protein",
  "gene_symbol": "MFSD14A",
  "gene": "UniProtKB:Q96MC6"
}